cytolytic granule [GO:0044194] (cellular component) References: PMID:11052265, PMID:12766758 Sources: GOC:jl Definition: A specialized secretory lysosome that is present in cells with cytolytic capability such as cytotoxic T lymphocytes and natural killer cells. Cytolytic granules mediate the storage and regulated excretion of lytic molecules for killing of target cells. Relationships: is a type of GO:0005764